{
  "gene_symbol": "CCDC184",
  "term_id": "UNKNOWN:0002",
  "gene": "UniProtKB:Q52MB2",
  "term_label": "Unknown biological process",
  "gene_name": "Coiled-coil domain-containing protein 184"
}